host caveola [GO:0044155] (cellular component) Relationships: is a type of GO:0033643; is part of host cell membrane [GO:0033644] Definition: A small pit, depression, or invagination, such as any of the minute pits or incuppings of the host cell membrane formed during pinocytosis, that communicates with the outside of a host cell and extends inward, indenting the host cytoplasm and the host cell membrane. Such caveolae may be pinched off to form free vesicles within the host cytoplasm. The host is defined as the larger of the organisms involved in a symbiotic interaction. Sources: GOC:rph